{
  "term_label": "type I interferon receptor binding",
  "gene": "UniProtKB:P05013",
  "gene_symbol": "IFNA6",
  "term_id": "GO:0005132",
  "gene_name": "Interferon alpha-6"
}